{
  "term_label": "C-C chemokine binding",
  "gene_symbol": "CXCR5",
  "term_id": "GO:0019957",
  "gene_name": "C-X-C chemokine receptor type 5",
  "gene": "UniProtKB:P32302"
}